{
  "gene_symbol": "DAP3",
  "gene": "UniProtKB:P51398",
  "gene_name": "Small ribosomal subunit protein mS29",
  "term_id": "GO:0003735",
  "term_label": "structural constituent of ribosome"
}